{
  "gene_name": "SH2B adapter protein 1",
  "gene_symbol": "SH2B1",
  "term_label": "plasma membrane",
  "term_id": "GO:0005886",
  "gene": "UniProtKB:Q9NRF2"
}